galanin receptor binding [GO:0031763] (molecular function) Sources: GOC:mah, GOC:nln Also known as: galanin receptor ligand Definition: Binding to a galanin receptor. Subtypes: GO:0031764, type 2 galanin receptor binding [GO:0031765], type 3 galanin receptor binding [GO:0031766] Relationships: is a type of neuropeptide receptor binding [GO:0071855]